{
  "term_id": "GO:0098703",
  "term_label": "calcium ion import across plasma membrane",
  "gene_name": "Voltage-dependent L-type calcium channel subunit alpha-1D",
  "gene_symbol": "CACNA1D",
  "gene": "UniProtKB:Q01668"
}